{
  "term_label": "regulation of potassium ion transmembrane transport",
  "term_id": "GO:1901379",
  "gene": "UniProtKB:Q8N608",
  "gene_name": "Inactive dipeptidyl peptidase 10",
  "gene_symbol": "DPP10"
}